{
  "gene_name": "Chromosome-associated kinesin KIF4B",
  "gene": "UniProtKB:Q2VIQ3",
  "term_id": "GO:0005875",
  "term_label": "microtubule associated complex",
  "gene_symbol": "KIF4B"
}